{
  "term_label": "Unknown molecular function",
  "gene": "UniProtKB:Q9Y3Y4",
  "term_id": "UNKNOWN:0001",
  "gene_symbol": "PYGO1",
  "gene_name": "Pygopus homolog 1"
}